{
  "gene_symbol": "CD3E",
  "term_label": "transmembrane signaling receptor activity",
  "term_id": "GO:0004888",
  "gene": "UniProtKB:P07766",
  "gene_name": "T-cell surface glycoprotein CD3 epsilon chain"
}